{
  "gene_symbol": "KLHDC3",
  "term_label": "cytoplasm",
  "gene": "UniProtKB:Q9BQ90",
  "gene_name": "Kelch domain-containing protein 3",
  "term_id": "GO:0005737"
}